{
  "term_id": "GO:0071818",
  "gene": "UniProtKB:P11441",
  "term_label": "BAT3 complex",
  "gene_symbol": "UBL4A",
  "gene_name": "Ubiquitin-like protein 4A"
}